{
  "gene": "UniProtKB:Q15022",
  "term_id": "GO:0005634",
  "gene_symbol": "SUZ12",
  "gene_name": "Polycomb protein SUZ12",
  "term_label": "nucleus"
}